regulation of phospholipase activity [GO:0010517] (biological process) Sources: GOC:BHF, GOC:dph, GOC:tb Subtypes: positive regulation of phospholipase activity [GO:0010518] Relationships: is a type of regulation of hydrolase activity [GO:0051336]; RO_0002211 phospholipase activity [GO:0004620] Definition: Any process that modulates the frequency, rate or extent of phospholipase activity, the hydrolysis of a phospholipid.